{
  "gene_symbol": "MAK16",
  "term_label": "maturation of LSU-rRNA",
  "gene": "UniProtKB:Q9BXY0",
  "term_id": "GO:0000470",
  "gene_name": "Protein MAK16 homolog"
}